{
  "term_label": "Unknown cellular component",
  "gene": "UniProtKB:Q9NU53",
  "term_id": "UNKNOWN:0003",
  "gene_symbol": "GINM1",
  "gene_name": "Glycoprotein integral membrane protein 1"
}